{
  "gene": "UniProtKB:Q53QZ3",
  "gene_symbol": "ARHGAP15",
  "term_id": "GO:0005096",
  "term_label": "GTPase activator activity",
  "gene_name": "Rho GTPase-activating protein 15"
}